{
  "gene_symbol": "G6PC2",
  "term_label": "membrane",
  "gene_name": "Glucose-6-phosphatase 2",
  "gene": "UniProtKB:Q9NQR9",
  "term_id": "GO:0016020"
}